{
  "term_label": "olfactory receptor activity",
  "gene_name": "Olfactory receptor 7E24",
  "gene": "UniProtKB:Q6IFN5",
  "gene_symbol": "OR7E24",
  "term_id": "GO:0004984"
}